dioxygenase activity [GO:0051213] (molecular function) References: PMID:1444267 Subtypes: oxidoreductase activity, acting on single donors with incorporation of molecular oxygen, incorporation of two atoms of oxygen [GO:0016702], 2-oxoglutarate-dependent dioxygenase activity [GO:0016706], oxidoreductase activity, acting on paired donors, with incorporation or reduction of molecular oxygen, NAD(P)H as one donor, and incorporation of two atoms of oxygen into one donor [GO:0016708], 1,2-dihydroxynaphthalene dioxygenase activity [GO:0018554], 3-butenylglucosinolate 2-hydroxylase activity [GO:0062131], alpha-ketoglutarate-dependent xanthine dioxygenase activity [GO:0097641] Relationships: is a type of oxidoreductase activity [GO:0016491] Definition: Catalysis of the incorporation of both atoms of molecular oxygen (O2) into the substrate.